siRNA-mediated post-transcriptional gene silencing [GO:0140766] (biological process) Relationships: is a type of regulatory ncRNA-mediated post-transcriptional gene silencing [GO:0035194] References: PMID:26372022 Definition: A post-transcriptional gene silencing pathway in which small interfering RNAs (siRNAs) elicit silencing of specific target genes. siRNAs are 21-23 nucleotide RNA duplexes that are fully complementary to their target mRNA. siRNAs can be exported and act in other cells, including in germline cells. Once incorporated into a RNA-induced silencing complex (RISC), siRNAs can downregulate gene expression by either of two posttranscriptional mechanisms: endonucleolytic cleavage of the mRNA or mRNA translational repression. siRNAs are present in lower animals and plants, but not found in mammals; whereas miRNAs are present in all the animals and in plants. Subtypes: siRNA-mediated gene silencing by inhibition of translation [GO:0070549], siRNA-mediated gene silencing by mRNA destabilization [GO:0090625] Also known as: siRNA-mediated gene silencing, gene silencing by siRNA, post-transcriptional gene silencing by siRNA, posttranscriptional gene silencing by siRNA, siRNA-mediated PTGS